D-aspartate transmembrane transport [GO:0070777] (BP) Definition: The process in which D-aspartate, the D-enantiomer of the anion of (2R)-2-aminobutanedioic acid  is transported across a lipid bilayer, from one side of a membrane to the other, by means of some agent such as a transporter or pore. Sources: GOC:mah, GOC:rph Relationships: is_a aspartate transmembrane transport [GO:0015810]; is a type of GO:0042940 Subtypes: D-aspartate import across plasma membrane [GO:0070779]